{
  "gene_symbol": "EVX2",
  "term_id": "GO:0006357",
  "gene_name": "Homeobox even-skipped homolog protein 2",
  "gene": "UniProtKB:Q03828",
  "term_label": "regulation of transcription by RNA polymerase II"
}